{
  "gene": "UniProtKB:P52306",
  "term_id": "UNKNOWN:0001",
  "gene_name": "Rap1 GTPase-GDP dissociation stimulator 1",
  "term_label": "Unknown molecular function",
  "gene_symbol": "RAP1GDS1"
}